{
  "gene_name": "Integrator complex subunit 12",
  "gene": "UniProtKB:Q96CB8",
  "gene_symbol": "INTS12",
  "term_label": "snRNA 3'-end processing",
  "term_id": "GO:0034472"
}